{
  "gene_name": "Actin-related protein 2_3 complex subunit 4",
  "gene": "UniProtKB:P59998",
  "term_label": "Arp2/3 complex-mediated actin nucleation",
  "gene_symbol": "ARPC4",
  "term_id": "GO:0034314"
}